{
  "term_label": "Unknown molecular function",
  "term_id": "UNKNOWN:0001",
  "gene_symbol": "OR8K3",
  "gene": "UniProtKB:Q8NH51",
  "gene_name": "Olfactory receptor 8K3"
}